{
  "gene_name": "Homeobox protein TGIF2LX",
  "term_id": "GO:0005634",
  "gene": "UniProtKB:Q8IUE1",
  "gene_symbol": "TGIF2LX",
  "term_label": "nucleus"
}